{
  "gene_name": "Dynein axonemal assembly factor 11",
  "gene": "UniProtKB:Q86X45",
  "term_id": "GO:0036158",
  "gene_symbol": "DNAAF11",
  "term_label": "outer dynein arm assembly"
}